carbohydrate derivative catabolic process [GO:1901136] (biological process) Definition: The chemical reactions and pathways resulting in the breakdown of carbohydrate derivative. Sources: GOC:TermGenie Also known as: carbohydrate derivative breakdown, carbohydrate derivative catabolism, carbohydrate derivative degradation Relationships: is a type of catabolic process [GO:0009056]; is_a GO:1901135 Subtypes: GO:0006026, GO:0006516, GO:0009050, lipopolysaccharide catabolic process [GO:0009104], ribonucleotide catabolic process [GO:0009261], GO:0009264, glycolipid catabolic process [GO:0019377], glyceraldehyde-3-phosphate catabolic process [GO:0019683], galactose catabolic process via UDP-galactose, Leloir pathway [GO:0033499], glycerol-3-phosphate catabolic process [GO:0046168], amino sugar catabolic process [GO:0046348], deoxyribose phosphate catabolic process [GO:0046386], diacetylchitobiose catabolic process [GO:0052777], teichoic acid catabolic process [GO:0070393], lipooligosaccharide catabolic process [GO:1901270], D-ribose 5-phosphate catabolic process [GO:1901279], GO:1901658, 6-sulfoquinovose(1-) catabolic process [GO:1902777], amylopectin catabolic process [GO:2000897], D-tagatose 6-phosphate catabolic process [GO:2001059]